{
  "term_label": "positive regulation of exocytosis",
  "gene_name": "Ras-related protein Rab-2B",
  "gene_symbol": "RAB2B",
  "term_id": "GO:0045921",
  "gene": "UniProtKB:Q8WUD1"
}